{
  "term_label": "protein stabilization",
  "gene_name": "Putative heat shock protein HSP 90-beta 2",
  "gene": "UniProtKB:Q58FF8",
  "gene_symbol": "HSP90AB2P",
  "term_id": "GO:0050821"
}